{
  "gene_name": "Transcription factor IIIB 50 kDa subunit",
  "term_id": "GO:0005634",
  "gene_symbol": "BRF2",
  "term_label": "nucleus",
  "gene": "UniProtKB:Q9HAW0"
}